{
  "gene_name": "Putative cytochrome c oxidase subunit 7A3, mitochondrial",
  "gene_symbol": "COX7A2P2",
  "term_id": "GO:0031966",
  "gene": "UniProtKB:O60397",
  "term_label": "mitochondrial membrane"
}